{
  "term_id": "GO:0005787",
  "gene_symbol": "SPCS1",
  "gene": "UniProtKB:Q9Y6A9",
  "term_label": "signal peptidase complex",
  "gene_name": "Signal peptidase complex subunit 1"
}